{
  "gene_symbol": "TUNAR",
  "term_label": "endoplasmic reticulum calcium ion homeostasis",
  "gene_name": "Protein TUNAR",
  "gene": "UniProtKB:A0A1B0GTB2",
  "term_id": "GO:0032469"
}